cell surface receptor signaling pathway involved in heart development [GO:0061311] (biological process) Also known as: cell surface receptor linked signaling pathway involved in heart development, cell surface receptor linked signalling pathway involved in heart development Subtypes: smoothened signaling pathway involved in regulation of secondary heart field cardioblast proliferation [GO:0003271], GO:0003306, fibroblast growth factor receptor signaling pathway involved in heart development [GO:0061313], Notch signaling involved in heart development [GO:0061314], GO:0071527 Definition: The series of molecular signals initiated by a ligand the binding to its receptor on the surface of a cell, which contributes to the progression of the heart over time. Relationships: is a type of cell surface receptor signaling pathway [GO:0007166]; BFO_0000050 heart development [GO:0007507] Sources: GOC:dph, GOC:mtg_heart, GOC:signaling